{
  "gene": "UniProtKB:P12268",
  "gene_name": "Inosine-5'-monophosphate dehydrogenase 2",
  "term_label": "GTP biosynthetic process",
  "gene_symbol": "IMPDH2",
  "term_id": "GO:0006183"
}